{
  "gene_name": "Zinc finger protein 521",
  "gene": "UniProtKB:Q96K83",
  "gene_symbol": "ZNF521",
  "term_id": "GO:0005634",
  "term_label": "nucleus"
}